{
  "term_id": "UNKNOWN:0002",
  "gene_symbol": "GLG1",
  "gene": "UniProtKB:Q92896",
  "term_label": "Unknown biological process",
  "gene_name": "Golgi apparatus protein 1"
}